{
  "gene_symbol": "IGFBP5",
  "gene": "UniProtKB:P24593",
  "gene_name": "Insulin-like growth factor-binding protein 5",
  "term_label": "extracellular space",
  "term_id": "GO:0005615"
}